{
  "gene_symbol": "MTCL1",
  "term_id": "GO:0000922",
  "term_label": "spindle pole",
  "gene_name": "Microtubule cross-linking factor 1",
  "gene": "UniProtKB:Q9Y4B5"
}